transferase activity, transferring nitrogenous groups [GO:0016769] (molecular function) Also known as: transferase activity, transferring other nitrogenous groups Definition: Catalysis of the transfer of a nitrogenous group from one compound (donor) to another (acceptor). Subtypes: GO:0002948, GPI-anchor transamidase activity [GO:0003923], transaminase activity [GO:0008483], GO:0033856, peptidyl-cysteine S-nitrosylase activity [GO:0035605], dATP(dGTP)-DNA purinetransferase activity [GO:0047839], oximinotransferase activity [GO:0050206] Relationships: is a type of transferase activity [GO:0016740] Sources: GOC:jl, ISBN:0198506732